{
  "gene": "UniProtKB:Q8IV13",
  "term_label": "cytoplasm",
  "gene_name": "Cyclin-J-like protein",
  "term_id": "GO:0005737",
  "gene_symbol": "CCNJL"
}